{
  "gene": "UniProtKB:Q96ER3",
  "gene_symbol": "SAAL1",
  "term_label": "Unknown molecular function",
  "gene_name": "Protein SAAL1",
  "term_id": "UNKNOWN:0001"
}